translation reinitiation [GO:0002188] (biological process) References: PMID:18056426, PMID:18765792 Relationships: is a type of GO:0002183 Definition: A gene-specific translational control mechanism where the small ribosomal subunit remains attached to the mRNA following termination of translation, then resumes scanning on the same mRNA molecule and initiates again at a downstream start site. Reinitiation depends on de novo recruitment of the ternary complex that is required to recognize the next AUG codon.